{
  "gene_symbol": "CSE1L",
  "term_id": "GO:0005635",
  "term_label": "nuclear envelope",
  "gene": "UniProtKB:P55060",
  "gene_name": "Exportin-2"
}